{
  "term_id": "GO:0007155",
  "gene_name": "Podoplanin",
  "term_label": "cell adhesion",
  "gene_symbol": "PDPN",
  "gene": "UniProtKB:Q86YL7"
}